{
  "gene_name": "Death effector domain-containing protein",
  "gene_symbol": "DEDD",
  "term_id": "GO:0005730",
  "term_label": "nucleolus",
  "gene": "UniProtKB:O75618"
}